UDP-rhamnose biosynthetic process [GO:0010253] (biological process) Definition: The chemical reactions and pathways resulting in the formation of UDP-L-rhamnose, a substance composed of rhamnose in glycosidic linkage with uridine diphosphate. References: PMID:15134748 Also known as: UDP-rhamnose anabolism, UDP-rhamnose biosynthesis, UDP-rhamnose formation, UDP-rhamnose synthesis Relationships: is a type of GO:0009226